{
  "term_id": "GO:0050252",
  "gene_name": "Acyl-CoA wax alcohol acyltransferase 2",
  "gene": "UniProtKB:Q6E213",
  "gene_symbol": "AWAT2",
  "term_label": "retinol O-fatty-acyltransferase activity"
}